{
  "term_label": "extracellular space",
  "gene": "UniProtKB:Q8N474",
  "gene_symbol": "SFRP1",
  "gene_name": "Secreted frizzled-related protein 1",
  "term_id": "GO:0005615"
}